{
  "gene_symbol": "NTRK3",
  "gene_name": "NT-3 growth factor receptor",
  "gene": "UniProtKB:Q16288",
  "term_label": "positive regulation of neuron projection development",
  "term_id": "GO:0010976"
}